{
  "term_id": "GO:0008284",
  "term_label": "positive regulation of cell population proliferation",
  "gene": "UniProtKB:Q9NP95",
  "gene_symbol": "FGF20",
  "gene_name": "Fibroblast growth factor 20"
}